guanosine pentaphosphate biosynthetic process [GO:0015973] (biological process) Also known as: guanosine pentaphosphate (5'-pppGpp-3') biosynthesis, guanosine pentaphosphate (5'-pppGpp-3') biosynthetic process, guanosine pentaphosphate anabolism, guanosine pentaphosphate biosynthesis, guanosine pentaphosphate formation, guanosine pentaphosphate synthesis Relationships: is a type of GO:0009152; is a type of GO:0015972; is a type of purine ribonucleoside bisphosphate biosynthetic process [GO:0034036] Sources: GOC:ai Definition: The chemical reactions and pathways resulting in the formation of guanine pentaphosphate (5'-pppGpp-3'), a derivative of guanine riboside with five phosphates.